negative regulation of CREB transcription factor activity [GO:0032792] (biological process) Definition: Any process that stops, prevents, or reduces the frequency, rate or extent of the activity of the transcription factor CREB. Relationships: is a type of GO:0043433 Also known as: inhibition of CREB transcription factor, CREB inhibitor Sources: GOC:dph, GOC:ecd, GOC:tb